spermine biosynthetic process [GO:0006597] (biological process) Relationships: is a type of GO:0006596; is a type of spermine metabolic process [GO:0008215] Sources: GOC:curators Also known as: spermine anabolism, spermine biosynthesis, spermine formation, spermine synthesis Definition: The chemical reactions and pathways resulting in the formation of spermine, a polybasic amine found in human sperm, in ribosomes and in some viruses and involved in nucleic acid packaging.